{
  "gene_symbol": "RFLNB",
  "term_label": "actin filament bundle",
  "gene_name": "Refilin-B",
  "term_id": "GO:0032432",
  "gene": "UniProtKB:Q8N5W9"
}